{
  "term_label": "peptidyl-prolyl cis-trans isomerase activity",
  "term_id": "GO:0003755",
  "gene_name": "Peptidyl-prolyl cis-trans isomerase F, mitochondrial",
  "gene": "UniProtKB:P30405",
  "gene_symbol": "PPIF"
}